borate transmembrane transport [GO:0035445] (BP) Also known as: borate membrane transport, boron transmembrane transport Definition: The process in which borate is transported across a membrane. Borate is the anion (BO3)3-; boron is a group 13 element, with properties which are borderline between metals and non-metals. Relationships: is a type of borate transport [GO:0046713]; is a type of transmembrane transport [GO:0055085] Sources: GOC:curators Subtypes: borate export across plasma membrane [GO:0140159] Note: Note that this term is not intended for use in annotating lateral movement within membranes.